{
  "gene": "UniProtKB:Q9H1V8",
  "term_label": "alanine transport",
  "gene_symbol": "SLC6A17",
  "term_id": "GO:0032328",
  "gene_name": "Sodium-dependent neutral amino acid transporter SLC6A17"
}